{
  "gene_symbol": "MOB1A",
  "gene": "UniProtKB:Q9H8S9",
  "term_label": "hippo signaling",
  "gene_name": "MOB kinase activator 1A",
  "term_id": "GO:0035329"
}